{
  "term_label": "guanyl-nucleotide exchange factor activity",
  "gene_name": "Ephexin-1",
  "term_id": "GO:0005085",
  "gene": "UniProtKB:Q8N5V2",
  "gene_symbol": "NGEF"
}